{
  "gene_name": "Olfactory receptor 2T6",
  "term_id": "GO:0050911",
  "term_label": "detection of chemical stimulus involved in sensory perception of smell",
  "gene_symbol": "OR2T6",
  "gene": "UniProtKB:Q8NHC8"
}